{
  "term_label": "double-strand break repair via homologous recombination",
  "gene_symbol": "SFR1",
  "gene": "UniProtKB:Q86XK3",
  "gene_name": "Swi5-dependent recombination DNA repair protein 1 homolog",
  "term_id": "GO:0000724"
}